{
  "gene": "UniProtKB:Q13621",
  "term_label": "chloride transmembrane transport",
  "gene_symbol": "SLC12A1",
  "term_id": "GO:1902476",
  "gene_name": "Solute carrier family 12 member 1"
}